transposable element silencing by siRNA-mediated DNA methylation [GO:0141010] (biological process) References: PMID:28633017, PMID:32381626, PMID:32719317, PMID:36570931 Definition: A transposable element silencing mechanism mediated by RNA-directed DNA methylation. RNA-directed DNA methylation is a gene silencing process in which small interfering RNAs (siRNAs) guide DNA methylation to the siRNA-generating genomic loci and other loci that are homologous to the siRNAs for de novo DNA methylation. This results in a heterochromatin assembly, a chromatin conformation that is refractory to transcription. Relationships: is a type of GO:0080188; is a type of transposable element silencing by heterochromatin formation [GO:0141005] Also known as: retrostransposon silencing by RdDM, transposable element silencing by siRNA-directed DNA methylation, retrotransposon silencing by siRNA-directed DNA methylation, retrotransposon silencing by RNA-directed DNA methylation